{
  "gene_name": "Condensin complex subunit 3",
  "gene_symbol": "NCAPG",
  "term_id": "GO:0000793",
  "gene": "UniProtKB:Q9BPX3",
  "term_label": "condensed chromosome"
}